{
  "gene_symbol": "SYS1",
  "gene": "UniProtKB:Q8N2H4",
  "gene_name": "Protein SYS1 homolog",
  "term_id": "GO:0005802",
  "term_label": "trans-Golgi network"
}